negative regulation of melanosome organization [GO:1903057] (biological process) References: PMID:24769727 Sources: GOC:BHF, GOC:TermGenie, GOC:rl, GO_REF:0000058 Also known as: down regulation of melanosome organisation, down regulation of melanosome organization, down-regulation of melanosome organisation, down-regulation of melanosome organization, downregulation of melanosome organisation, downregulation of melanosome organization, negative regulation of melanosome organisation, inhibition of melanosome organisation, inhibition of melanosome organization, down regulation of melanosome organization and biogenesis, down-regulation of melanosome organization and biogenesis, downregulation of melanosome organization and biogenesis, inhibition of melanosome organization and biogenesis, negative regulation of melanosome organization and biogenesis Relationships: is a type of negative regulation of organelle organization [GO:0010639]; is a type of regulation of melanosome organization [GO:1903056]; negatively regulates melanosome organization [GO:0032438] Note: Lack of the transcription factor Zeb2 Q9R0G7 leads to spherical melanosomes with irregular borders, in contrast to the rod-shaped melanosomes of ZEB2MCWT hair follicles. Definition: Any process that stops, prevents or reduces the frequency, rate or extent of melanosome organization.